{
  "gene_symbol": "IQCE",
  "gene_name": "IQ domain-containing protein E",
  "term_id": "UNKNOWN:0002",
  "term_label": "Unknown biological process",
  "gene": "UniProtKB:Q6IPM2"
}